{
  "gene_symbol": "LOXHD1",
  "gene": "UniProtKB:Q8IVV2",
  "term_label": "Unknown molecular function",
  "gene_name": "Lipoxygenase homology domain-containing protein 1",
  "term_id": "UNKNOWN:0001"
}